{
  "term_label": "N-acetylglucosamine metabolic process",
  "term_id": "GO:0006044",
  "gene": "UniProtKB:Q09327",
  "gene_symbol": "MGAT3",
  "gene_name": "Beta-1,4-mannosyl-glycoprotein 4-beta-N-acetylglucosaminyltransferase"
}